{
  "gene_name": "Coiled-coil domain-containing protein 171",
  "term_id": "UNKNOWN:0001",
  "gene_symbol": "CCDC171",
  "term_label": "Unknown molecular function",
  "gene": "UniProtKB:Q6TFL3"
}